{
  "gene_name": "Oncoprotein-induced transcript 3 protein",
  "gene_symbol": "OIT3",
  "gene": "UniProtKB:Q8WWZ8",
  "term_label": "cell surface",
  "term_id": "GO:0009986"
}